{
  "term_id": "GO:0001570",
  "gene_symbol": "NRP1",
  "gene": "UniProtKB:O14786",
  "gene_name": "Neuropilin-1",
  "term_label": "vasculogenesis"
}